{
  "term_label": "mitochondrial tRNA wobble uridine modification",
  "gene_symbol": "MTO1",
  "gene": "UniProtKB:Q9Y2Z2",
  "term_id": "GO:0070899",
  "gene_name": "Protein MTO1 homolog, mitochondrial"
}